{
  "term_label": "GTPase activator activity",
  "term_id": "GO:0005096",
  "gene_symbol": "GIT2",
  "gene_name": "ARF GTPase-activating protein GIT2",
  "gene": "UniProtKB:Q14161"
}